RIG-I signaling pathway [GO:0039529] (biological process) Also known as: DDX58 signaling pathway, RIG-I signalling pathway, RIG-I-like receptor (RLR) signaling pathway, RIG-like helicase signaling pathway, RIG-like receptor signaling pathway, RLH signaling pathway, RLR signaling pathway, retinoic acid inducible gene I signaling pathway References: PMID:17328678, PMID:19620789, PMID:21435580, PMID:25579795 Sources: GOC:bf Relationships: is a type of cytoplasmic pattern recognition receptor signaling pathway [GO:0002753] Definition: The series of molecular signals initiated by the binding ssRNA or dsRNA from another organism to the cytoplasmic pattern recognition receptor (PRR) RIG-1 (also known as DDX58). RIG-I detects RNA synthesized during viral replication or shed by non-viral pathogens, and triggers a signaling pathway to protect the host against infection, for example by inducing the expression of cytokines. Regulation: regulated by regulation of RIG-I signaling pathway [GO:0039535]; RO_0002212 by negative regulation of RIG-I signaling pathway [GO:0039536]; positively regulated by GO:1900246